protein flavinylation [GO:0017013] (biological process) Definition: The addition of a flavin group to a protein amino acid. Also known as: protein amino acid flavinylation Relationships: is a type of protein modification process [GO:0036211] Sources: GOC:ai